{
  "term_label": "polysaccharide biosynthetic process",
  "term_id": "GO:0000271",
  "gene_symbol": "HAS1",
  "gene": "UniProtKB:Q92839",
  "gene_name": "Hyaluronan synthase 1"
}